{
  "gene_symbol": "ESYT2",
  "term_id": "UNKNOWN:0002",
  "gene_name": "Extended synaptotagmin-2",
  "term_label": "Unknown biological process",
  "gene": "UniProtKB:A0FGR8"
}